{
  "gene_name": "Peroxisome proliferator-activated receptor gamma coactivator-related protein 1",
  "term_label": "nucleus",
  "term_id": "GO:0005634",
  "gene": "UniProtKB:Q5VV67",
  "gene_symbol": "PPRC1"
}